{
  "gene_symbol": "SPATA17",
  "gene_name": "Spermatogenesis-associated protein 17",
  "term_id": "UNKNOWN:0001",
  "gene": "UniProtKB:Q96L03",
  "term_label": "Unknown molecular function"
}